{
  "gene_symbol": "OSTF1",
  "gene_name": "Osteoclast-stimulating factor 1",
  "term_label": "Unknown cellular component",
  "gene": "UniProtKB:Q92882",
  "term_id": "UNKNOWN:0003"
}